{
  "gene": "UniProtKB:Q96JQ5",
  "gene_name": "Membrane-spanning 4-domains subfamily A member 4A",
  "term_id": "GO:0005794",
  "gene_symbol": "MS4A4A",
  "term_label": "Golgi apparatus"
}